{
  "gene_symbol": "KIF3C",
  "term_label": "ATP hydrolysis activity",
  "gene_name": "Kinesin-like protein KIF3C",
  "term_id": "GO:0016887",
  "gene": "UniProtKB:O14782"
}